{
  "term_id": "GO:0050839",
  "gene": "UniProtKB:Q9Y5E5",
  "term_label": "cell adhesion molecule binding",
  "gene_name": "Protocadherin beta-4",
  "gene_symbol": "PCDHB4"
}